negative regulation of prostaglandin secretion [GO:0032307] (biological process) Relationships: is a type of negative regulation of icosanoid secretion [GO:0032304]; is a type of regulation of prostaglandin secretion [GO:0032306]; is a type of GO:1903531; RO_0002212 prostaglandin secretion [GO:0032310] Sources: GOC:mah Also known as: down regulation of prostaglandin secretion, down-regulation of prostaglandin secretion, downregulation of prostaglandin secretion, inhibition of prostaglandin secretion, negative regulation of prostacyclin secretion Definition: Any process that stops, prevents, or reduces the frequency, rate or extent of the regulated release of a prostaglandin from a cell.